{
  "term_label": "protein K11-linked ubiquitination",
  "gene_name": "Ubiquitin-conjugating enzyme E2 D4",
  "term_id": "GO:0070979",
  "gene": "UniProtKB:Q9Y2X8",
  "gene_symbol": "UBE2D4"
}